negative regulation of skeletal muscle fiber differentiation [GO:1902810] (biological process) Subtypes: GO:2001036 Definition: Any process that stops, prevents or reduces the frequency, rate or extent of skeletal muscle fiber differentiation. Also known as: down regulation of skeletal muscle fiber differentiation, down-regulation of skeletal muscle fiber differentiation, downregulation of skeletal muscle fiber differentiation, inhibition of skeletal muscle fiber differentiation References: PMID:17879321 Sources: GOC:TermGenie, GOC:mr, GO_REF:0000058 Relationships: is a type of negative regulation of myotube differentiation [GO:0010832]; is a type of regulation of skeletal muscle fiber differentiation [GO:1902809]; is_a negative regulation of skeletal muscle cell differentiation [GO:2001015]; RO_0002212 GO:0098528